{
  "gene": "UniProtKB:P56730",
  "gene_symbol": "PRSS12",
  "gene_name": "Neurotrypsin",
  "term_label": "synaptic cleft",
  "term_id": "GO:0043083"
}